{
  "term_id": "GO:0008285",
  "term_label": "negative regulation of cell population proliferation",
  "gene_symbol": "NUPR1",
  "gene_name": "Nuclear protein 1",
  "gene": "UniProtKB:O60356"
}